{
  "gene": "UniProtKB:O43897",
  "term_id": "GO:0005615",
  "gene_symbol": "TLL1",
  "gene_name": "Tolloid-like protein 1",
  "term_label": "extracellular space"
}